cleavage of bicistronic rRNA transcript (SSU-rRNA, LSU-rRNA) [GO:0000450] (biological process) Sources: GOC:curators Definition: Endonucleolytic cleavage of pre-rRNAs originally produced as a bicistronic rRNA transcript that contains the SSU-rRNA and the LSU-rRNA in that order from 5' to 3' along the primary transcript. Primary ribosomal RNA transcripts with two genes in this order are produced in Archaeal species. Relationships: is a type of GO:0006364